{
  "term_id": "GO:0019901",
  "gene": "UniProtKB:Q03135",
  "term_label": "protein kinase binding",
  "gene_symbol": "CAV1",
  "gene_name": "Caveolin-1"
}